excitation of vasomotor center by carotid body chemoreceptor signaling [GO:0003041] (biological process) Sources: GOC:mtg_cardio Definition: The process in which the molecular signal from a carotid body is relayed to the vasomotor center, causing it to signal an increase arterial pressure. Relationships: is a type of excitation of vasomotor center by chemoreceptor signaling [GO:0002008]; is part of regulation of systemic arterial blood pressure by carotid body chemoreceptor signaling [GO:0003027] Also known as: excitation of vasomotor center by carotid body chemoreceptor signalling